chloroplast protein-transporting ATPase activity [GO:0016464] (molecular function) Also known as: AAA chloroplast protein-transporting ATPase, ATPase-coupled chloroplast protein transporter activity Definition: Enables the transfer of a solute or solutes from one side of a membrane to the other according to the reaction: ATP + H2O = ADP + phosphate; drives the transport of proteins into the chloroplast stroma. Relationships: is a type of protein-transporting ATPase activity [GO:0015450] Sources: EC:7.4.2.4